fructan beta-fructosidase activity [GO:0051669] (MF) Also known as: exo-beta-D-fructosidase activity, exo-beta-fructosidase activity, fructan b-fructosidase activity, fructan exohydrolase activity, polysaccharide beta-fructofuranosidase activity, beta-D-fructan fructohydrolase activity, fructanase activity Sources: EC:3.2.1.80 Definition: Catalysis of the hydrolysis of terminal, non-reducing 2,1- and 2,6-linked beta-D-fructofuranose residues in fructans. Relationships: is a type of hydrolase activity, hydrolyzing O-glycosyl compounds [GO:0004553]